{
  "gene_name": "STAGA complex 65 subunit gamma",
  "term_id": "UNKNOWN:0003",
  "term_label": "Unknown cellular component",
  "gene": "UniProtKB:O94864",
  "gene_symbol": "SUPT7L"
}